{
  "term_id": "GO:0019901",
  "gene_symbol": "POTEKP",
  "term_label": "protein kinase binding",
  "gene_name": "Putative beta-actin-like protein 3",
  "gene": "UniProtKB:Q9BYX7"
}